{
  "term_label": "nucleus",
  "gene_name": "Activating transcription factor 7-interacting protein 1",
  "term_id": "GO:0005634",
  "gene": "UniProtKB:Q6VMQ6",
  "gene_symbol": "ATF7IP"
}